{
  "term_label": "positive regulation of growth hormone secretion",
  "gene": "UniProtKB:Q9UBU3",
  "term_id": "GO:0060124",
  "gene_symbol": "GHRL",
  "gene_name": "Appetite-regulating hormone"
}